{
  "gene": "UniProtKB:Q8IW41",
  "term_id": "GO:0005516",
  "gene_name": "MAP kinase-activated protein kinase 5",
  "gene_symbol": "MAPKAPK5",
  "term_label": "calmodulin binding"
}